{
  "gene_symbol": "OR52E5",
  "gene": "UniProtKB:Q8NH55",
  "term_label": "plasma membrane",
  "gene_name": "Olfactory receptor 52E5",
  "term_id": "GO:0005886"
}